positive regulation of translational initiation in response to stress [GO:0032058] (biological process) Also known as: up regulation of translation initiation in response to stress, up-regulation of translation initiation in response to stress, upregulation of translation initiation in response to stress, activation of translation initiation in response to stress, stimulation of translation initiation in response to stress Definition: Any process that activates or increases the frequency, rate or extent of translation initiation as a result of a stimulus indicating the organism is under stress. Relationships: is a type of positive regulation of translational initiation [GO:0045948]; is part of GO:0006950 Subtypes: GO:0032064, positive regulation of translation initiation in response to endoplasmic reticulum stress [GO:0036494], positive regulation of translational initiation in response to starvation [GO:0071264] Sources: GOC:mah